{
  "gene_symbol": "GAGE12H",
  "gene": "UniProtKB:A6NDE8",
  "term_id": "UNKNOWN:0002",
  "term_label": "Unknown biological process",
  "gene_name": "G antigen 12H"
}